{
  "gene_symbol": "RFXANK",
  "term_label": "Unknown molecular function",
  "term_id": "UNKNOWN:0001",
  "gene": "UniProtKB:O14593",
  "gene_name": "DNA-binding protein RFXANK"
}